{
  "gene": "UniProtKB:Q9GZT9",
  "gene_name": "Egl nine homolog 1",
  "gene_symbol": "EGLN1",
  "term_label": "cellular response to hypoxia",
  "term_id": "GO:0071456"
}